{
  "gene_name": "Cadherin-related family member 3",
  "gene": "UniProtKB:Q6ZTQ4",
  "gene_symbol": "CDHR3",
  "term_id": "GO:0008013",
  "term_label": "beta-catenin binding"
}